{
  "gene": "UniProtKB:Q86VZ1",
  "term_id": "GO:0005886",
  "term_label": "plasma membrane",
  "gene_name": "P2Y purinoceptor 8",
  "gene_symbol": "P2RY8"
}